chemokine (C-C motif) ligand 6 production [GO:0035530] (biological process) Definition: The appearance of chemokine (C-C motif) ligand 6 (CCL6) due to biosynthesis or secretion following a cellular stimulus, resulting in an increase in its intracellular or extracellular levels. References: PMID:19812544 Sources: GOC:add Also known as: CCL6 production Relationships: is a type of chemokine production [GO:0032602] Regulation: regulated by regulation of chemokine (C-C motif) ligand 6 production [GO:0035531]; negatively regulated by negative regulation of chemokine (C-C motif) ligand 6 production [GO:0035532]; positively regulated by positive regulation of chemokine (C-C motif) ligand 6 production [GO:0035533]